{
  "gene_name": "Immunoglobulin superfamily member 11",
  "term_id": "UNKNOWN:0002",
  "term_label": "Unknown biological process",
  "gene": "UniProtKB:Q5DX21",
  "gene_symbol": "IGSF11"
}